{
  "gene_symbol": "CAMKMT",
  "term_id": "GO:0018025",
  "term_label": "calmodulin-lysine N-methyltransferase activity",
  "gene_name": "Calmodulin-lysine N-methyltransferase",
  "gene": "UniProtKB:Q7Z624"
}